{
  "gene": "UniProtKB:Q92614",
  "gene_name": "Unconventional myosin-XVIIIa",
  "term_label": "actin filament binding",
  "term_id": "GO:0051015",
  "gene_symbol": "MYO18A"
}